{
  "term_id": "GO:0030681",
  "gene_symbol": "RPP38",
  "gene_name": "Ribonuclease P protein subunit p38",
  "term_label": "multimeric ribonuclease P complex",
  "gene": "UniProtKB:P78345"
}